{
  "gene_symbol": "TRAV30",
  "term_label": "Unknown cellular component",
  "gene": "UniProtKB:A0A087WSZ9",
  "term_id": "UNKNOWN:0003",
  "gene_name": "T cell receptor alpha variable 30"
}